mannosyl-inositol phosphorylceramide biosynthetic process [GO:0051999] (biological process) Relationships: is a type of mannosyl-inositol phosphorylceramide metabolic process [GO:0006675]; is a type of glycosphingolipid biosynthetic process [GO:0006688]; is a type of phospholipid biosynthetic process [GO:0008654] Also known as: MIPC biosynthetic process, mannose inositol phosphoceramide biosynthetic process, mannose-inositol-P-ceramide (MIPC) biosynthetic process, mannosyl-inositol phosphorylceramide anabolism, mannosyl-inositol phosphorylceramide biosynthesis, mannosyl-inositol phosphorylceramide formation, mannosyl-inositol phosphorylceramide synthesis Sources: GOC:ai Definition: The chemical reactions and pathways resulting in the formation of mannosyl-inositol phosphorylceramide, any lipid with a phosphodiester bridge between an inositol residue and the ceramide group which contains a phosphoryl (-P(O)=) groups and a mannose derivative.